{
  "term_label": "cell projection",
  "gene_name": "Alpha-actinin-2",
  "gene": "UniProtKB:P35609",
  "gene_symbol": "ACTN2",
  "term_id": "GO:0042995"
}